L-tryptophan 2,3-dioxygenase activity [GO:0004833] (molecular function) Relationships: is a type of oxidoreductase activity, acting on single donors with incorporation of molecular oxygen, incorporation of two atoms of oxygen [GO:0016702] Definition: Catalysis of the reaction: L-tryptophan + O2 = N-formyl-L-kynurenine. Also known as: indolamine 2,3-dioxygenase activity, tryptophan oxygenase activity, tryptophan peroxidase activity, tryptophan pyrrolase activity, indoleamine-pyrrole 2,3-dioxygenase activity, tryptophan 2,3-dioxygenase activity, L-tryptophan pyrrolase activity, L-tryptophan:oxygen 2,3-oxidoreductase (decyclizing), TDO, tryptamin 2,3-dioxygenase activity, tryptamine 2,3-dioxygenase activity Sources: EC:1.13.11.11